high molecular weight B cell growth factor receptor activity [GO:0030373] (molecular function) Definition: Combining with a high molecular weight B cell growth factor and transmitting the signal to initiate a change in cell activity. Also known as: HMW-BCGF receptor, high molecular weight B lymphocyte growth factor receptor activity, high molecular weight B-cell growth factor receptor activity, high molecular weight B-lymphocyte growth factor receptor activity Relationships: is a type of GO:0038023 References: PMID:2681271 Sources: GOC:ai, GOC:signaling